{
  "gene_symbol": "RAB1B",
  "term_id": "GO:0006886",
  "term_label": "intracellular protein transport",
  "gene": "UniProtKB:Q9H0U4",
  "gene_name": "Ras-related protein Rab-1B"
}